advanced glycation end-product binding [GO:1904599] (molecular function) Definition: Binding to advanced glycation end-product. Relationships: is a type of carbohydrate derivative binding [GO:0097367] References: PMID:1650387 Sources: GOC:TermGenie, GOC:krc, GO_REF:0000067